COPI-coated vesicle [GO:0030137] (cellular component) Definition: A vesicle with a coat formed of the COPI coat complex proteins. COPI-coated vesicles are found associated with Golgi membranes at steady state, are involved in Golgi to endoplasmic reticulum (retrograde) vesicle transport, and possibly also in intra-Golgi transport. Also known as: coatomer Relationships: is a type of Golgi-associated vesicle [GO:0005798]; is a type of GO:0030135 Subtypes: COPI-coated Golgi to ER transport vesicle [GO:0030142], COPI-coated inter-Golgi transport vesicle [GO:0030143] References: PMID:11252894 Sources: GOC:mah